{
  "gene_symbol": "SNAPIN",
  "gene_name": "SNARE-associated protein Snapin",
  "gene": "UniProtKB:O95295",
  "term_id": "GO:0008333",
  "term_label": "endosome to lysosome transport"
}